{
  "gene_name": "AP-4 complex accessory subunit RUSC1",
  "gene_symbol": "RUSC1",
  "gene": "UniProtKB:Q9BVN2",
  "term_id": "UNKNOWN:0001",
  "term_label": "Unknown molecular function"
}